ribonucleoside triphosphate catabolic process [GO:0009203] (biological process) Definition: The chemical reactions and pathways resulting in the breakdown of a ribonucleoside triphosphate, a compound consisting of a nucleobase linked to a ribose sugar esterified with triphosphate on the sugar. Sources: GOC:go_curators, ISBN:0198506732 Also known as: ribonucleoside triphosphate breakdown, ribonucleoside triphosphate catabolism, ribonucleoside triphosphate degradation Subtypes: purine ribonucleoside triphosphate catabolic process [GO:0009207], pyrimidine ribonucleoside triphosphate catabolic process [GO:0009210] Relationships: is a type of GO:0009143